JAK pathway signal transduction adaptor activity [GO:0008269] (molecular function) Sources: GOC:mtg_MIT_16mar07 Definition: The binding activity of a molecule that brings together two molecules of the JAK signal transduction pathway, permitting them to function in a coordinated way. Relationships: is a type of signaling adaptor activity [GO:0035591]; is part of regulation of receptor signaling pathway via JAK-STAT [GO:0046425]